axial mesodermal cell fate commitment [GO:0048322] (biological process) Relationships: is a type of mesodermal cell fate commitment [GO:0001710]; is part of axial mesodermal cell differentiation [GO:0048321] Definition: The process in which a cell becomes committed to become an axial mesoderm cell. Also known as: axial mesoderm cell fate commitment Sources: GOC:dgh